{
  "gene_name": "Bcl-2-like protein 11",
  "gene": "UniProtKB:O43521",
  "gene_symbol": "BCL2L11",
  "term_id": "GO:0005739",
  "term_label": "mitochondrion"
}